antimicrobial peptide production [GO:0002775] (biological process) Regulation: positively regulated by positive regulation of antimicrobial peptide production [GO:0002225]; regulated by GO:0002784; negatively regulated by negative regulation of antimicrobial peptide production [GO:0002785] Subtypes: antibacterial peptide production [GO:0002778], antifungal peptide production [GO:0002781] Note: Note that this term is in the subset of terms that should not be used for direct gene product annotation. Instead, select one of the 'regulation' children terms. Definition: The synthesis or release of an antimicrobial peptide during an immune response, resulting in an increase in intracellular or extracellular levels. Such peptides may have protective properties against bacteria, fungi, viruses, or protozoa. References: PMID:11807545, PMID:15638771 Sources: GOC:add, ISBN:0781735149 Relationships: is a type of production of molecular mediator of immune response [GO:0002440]; is part of GO:0061844